{
  "gene_name": "Vascular endothelial growth factor receptor 1",
  "term_label": "positive regulation of cell population proliferation",
  "gene_symbol": "FLT1",
  "gene": "UniProtKB:P17948",
  "term_id": "GO:0008284"
}